{
  "term_label": "protein localization to phagophore assembly site",
  "term_id": "GO:0034497",
  "gene_name": "Autophagy-related protein 9A",
  "gene": "UniProtKB:Q7Z3C6",
  "gene_symbol": "ATG9A"
}